{
  "term_label": "positive regulation of immune response",
  "term_id": "GO:0050778",
  "gene_symbol": "HLA-DQA1",
  "gene": "UniProtKB:P01909",
  "gene_name": "HLA class II histocompatibility antigen, DQ alpha 1 chain"
}